{
  "gene": "UniProtKB:Q8NGY2",
  "gene_symbol": "OR6K2",
  "term_id": "GO:0005549",
  "term_label": "odorant binding",
  "gene_name": "Olfactory receptor 6K2"
}